{
  "term_id": "GO:0050911",
  "gene_name": "Olfactory receptor 13C2",
  "gene_symbol": "OR13C2",
  "gene": "UniProtKB:Q8NGS9",
  "term_label": "detection of chemical stimulus involved in sensory perception of smell"
}